{
  "gene": "UniProtKB:B4DU55",
  "gene_name": "Zinc finger protein 879",
  "gene_symbol": "ZNF879",
  "term_id": "GO:0006357",
  "term_label": "regulation of transcription by RNA polymerase II"
}